{
  "term_id": "GO:0016020",
  "gene_symbol": "ATP6V0B",
  "term_label": "membrane",
  "gene_name": "V-type proton ATPase 21 kDa proteolipid subunit c''",
  "gene": "UniProtKB:Q99437"
}